leg disc morphogenesis [GO:0007478] (biological process) Definition: The process in which the anatomical structures derived from the leg disc are generated and organized. This includes the transformation of a leg imaginal disc from a monolayered epithelium in the larvae of holometabolous insects into recognizable adult structures including the leg, coxa and ventral thoracic pleura. Relationships: is a type of GO:0007560; is part of GO:0035218 Also known as: leg disc metamorphosis Sources: GOC:bf, ISBN:0879694238